cerebellar granule cell differentiation [GO:0021707] (biological process) Definition: The process in which neuroblasts acquire specialized structural and/or functional features that characterize the mature cerebellar granule cell. Differentiation includes the processes involved in commitment of a neuroblast to a granule cell fate. A granule cell is a glutamatergic interneuron found in the cerebellar cortex. References: PMID:15157725 Sources: GOC:cls, GOC:dgh, GOC:dph, GOC:jid, GO_REF:0000021 Relationships: is a type of cell differentiation in hindbrain [GO:0021533]; is a type of GO:0021953; is a type of glutamatergic neuron differentiation [GO:1905962]; is part of cerebellar granular layer formation [GO:0021684]